cargo loading involved in clathrin-dependent endocytosis [GO:0099043] (biological process) Definition: Formation of a macromolecular complex during clathrin-dependent endocytosis that connects the assembling clathrin coat to the proteins and/or lipoproteins to be transported in an endocytic vesicle. This complex includes a receptor and an adaptor protein that links the receptor to the clathrin coat. References: PMID:21779028 Sources: GOC:dos, GOC:lb, GOC:vw Relationships: is a type of clathrin-coated vesicle cargo loading [GO:0035652]; is part of clathrin-dependent endocytosis [GO:0072583]